{
  "term_id": "GO:0000786",
  "gene_symbol": "H3-5",
  "term_label": "nucleosome",
  "gene": "UniProtKB:Q6NXT2",
  "gene_name": "Histone H3.3C"
}